2-(R)-hydroxypropyl-CoM dehydrogenase activity [GO:0050574] (molecular function) Sources: EC:1.1.1.268, RHEA:13249 Also known as: 2-(2-(R)-hydroxypropylthio)ethanesulfonate dehydrogenase activity, 2-[2-(R)-hydroxypropylthio]ethanesulfonate:NAD+ oxidoreductase activity Definition: Catalysis of the reaction: 2-(R)-hydroxypropyl-coenzyme M + NAD+ = 2-oxopropyl-coenzyme M + H+ + NADH. Relationships: is a type of oxidoreductase activity, acting on the CH-OH group of donors, NAD or NADP as acceptor [GO:0016616]